{
  "gene": "UniProtKB:A2RUB1",
  "term_id": "GO:0005737",
  "gene_symbol": "MEIOC",
  "gene_name": "Meiosis-specific coiled-coil domain-containing protein MEIOC",
  "term_label": "cytoplasm"
}